{
  "gene": "UniProtKB:Q6ZQT7",
  "gene_name": "Putative uncharacterized protein FLJ44672",
  "gene_symbol": "Q6ZQT7",
  "term_id": "UNKNOWN:0001",
  "term_label": "Unknown molecular function"
}